bitter taste receptor activity [GO:0033038] (molecular function) Definition: Combining with soluble bitter compounds to initiate a change in cell activity. These receptors are responsible for the sense of bitter taste. Sources: GOC:mah Subtypes: GPCR bitter taste receptor activity [GO:0090682] Relationships: is a type of taste receptor activity [GO:0008527]; is part of GO:0001580